meiotic sister chromatid centromere separation [GO:0051756] (biological process) Relationships: is a type of GO:0034510; is a type of GO:1903046; is part of meiotic sister chromatid segregation [GO:0045144]; is part of meiotic sister chromatid separation [GO:0051757] References: PMID:14730319, PMID:16325576 Sources: GOC:ai Definition: The cell cycle process in which the centromeres of sister chromatids are physically detached from each other during meiosis.